{
  "gene_symbol": "RING1",
  "gene_name": "E3 ubiquitin-protein ligase RING1",
  "gene": "UniProtKB:Q06587",
  "term_id": "GO:0000151",
  "term_label": "ubiquitin ligase complex"
}